{
  "term_id": "GO:0015937",
  "gene_name": "Pantothenate kinase 1",
  "term_label": "coenzyme A biosynthetic process",
  "gene_symbol": "PANK1",
  "gene": "UniProtKB:Q8TE04"
}